{
  "gene": "UniProtKB:Q8N3F8",
  "gene_symbol": "MICALL1",
  "term_id": "GO:0030036",
  "term_label": "actin cytoskeleton organization",
  "gene_name": "MICAL-like protein 1"
}